{
  "term_id": "GO:0050679",
  "gene_symbol": "EGFR",
  "term_label": "positive regulation of epithelial cell proliferation",
  "gene_name": "Epidermal growth factor receptor",
  "gene": "UniProtKB:P00533"
}